roof plate formation [GO:0021509] (biological process) Relationships: is a type of anatomical structure formation involved in morphogenesis [GO:0048646]; is part of neural tube formation [GO:0001841] References: PMID:15936325 Sources: GOC:cls, GOC:dgh, GOC:dph, GOC:jid, GO_REF:0000021 Definition: The formation of a single row of glia at the dorsal midline of the developing neural tube. This region provides inductive signals for the specification of neuronal cell types and of the specification of neural crest cells. The cells comprising the roof plate are the precursors to radial glial cells.